transforming growth factor beta receptor activity [GO:0005024] (molecular function) Relationships: is a type of transmembrane receptor protein serine/threonine kinase activity [GO:0004675] Sources: GOC:mah, GOC:signaling Subtypes: transforming growth factor beta receptor activity, type I [GO:0005025], transforming growth factor beta receptor activity, type II [GO:0005026], transforming growth factor beta receptor activity, type III [GO:0070123] Note: Note that this term represents an activity and not a gene product, and should only be used when the receptor binds the ligand TGFbeta. For binding to other growth factors, consider annotating to terms under 'transmembrane signaling receptor activity ; GO:0004888. Also known as: TGF-beta receptor activity, TGFbeta receptor activity, TGFbeta-activated receptor activity, TGFbetaR, transforming growth factor beta-activated receptor activity Definition: Combining with a transforming growth factor beta (TGFbeta) and transmitting the signal from one side of the membrane to the other to initiate a change in cell activity by catalysis of the reaction: ATP protein serine = ADP + protein serine phosphate, and ATP + protein threonine = ADP + protein threonine phosphate.